{
  "term_id": "GO:0090263",
  "gene_name": "Transmembrane protein 198",
  "term_label": "positive regulation of canonical Wnt signaling pathway",
  "gene": "UniProtKB:Q66K66",
  "gene_symbol": "TMEM198"
}